exochitinase activity [GO:0035885] (molecular function) Definition: Catalysis of the hydrolysis of terminal 1,4-beta-linkages of N-acetyl-D-glucosamine (GlcNAc) polymers of chitin and chitodextrins. Typically, exochitinases progressively cleave off two subunits from the reducing or non-reducing ends of the chitin chain. Relationships: is a type of chitinase activity [GO:0004568] References: PMID:11468293, PMID:16298970, PMID:21390509 Sources: GOC:bf, GOC:kah, GOC:pde